negative regulation of unidimensional cell growth [GO:0051511] (biological process) Subtypes: negative regulation of monopolar cell growth [GO:0051514], negative regulation of bipolar cell growth [GO:0051517] Also known as: down regulation of unidimensional cell growth, down-regulation of unidimensional cell growth, downregulation of unidimensional cell growth, inhibition of unidimensional cell growth, negative regulation of cell elongation Relationships: is a type of negative regulation of cell morphogenesis [GO:0010771]; is a type of negative regulation of cell growth [GO:0030308]; is a type of negative regulation of developmental growth [GO:0048640]; is a type of regulation of unidimensional cell growth [GO:0051510]; negatively regulates unidimensional cell growth [GO:0009826] Sources: GOC:ai Definition: Any process that stops, prevents, or reduces the frequency, rate or extent of unidimensional cell growth, the process in which a cell irreversibly increases in size in one [spatial] dimension or along one axis.